{
  "term_label": "regulation of transcription by RNA polymerase II",
  "gene": "UniProtKB:O60806",
  "gene_symbol": "TBX19",
  "term_id": "GO:0006357",
  "gene_name": "T-box transcription factor TBX19"
}